{
  "gene_name": "Methylated-DNA--protein-cysteine methyltransferase",
  "term_id": "GO:0003908",
  "gene": "UniProtKB:P16455",
  "term_label": "methylated-DNA-[protein]-cysteine S-methyltransferase activity",
  "gene_symbol": "MGMT"
}